{
  "gene_symbol": "IGLON5",
  "term_label": "regulation of synapse assembly",
  "gene_name": "IgLON family member 5",
  "gene": "UniProtKB:A6NGN9",
  "term_id": "GO:0051963"
}